{
  "term_label": "extracellular space",
  "gene_name": "Phospholipase A1 member A",
  "gene": "UniProtKB:Q53H76",
  "gene_symbol": "PLA1A",
  "term_id": "GO:0005615"
}